{
  "term_label": "DNA-binding transcription activator activity, RNA polymerase II-specific",
  "term_id": "GO:0001228",
  "gene": "UniProtKB:Q12800",
  "gene_symbol": "TFCP2",
  "gene_name": "Alpha-globin transcription factor CP2"
}